{
  "term_label": "Unknown molecular function",
  "gene_symbol": "MEX3B",
  "term_id": "UNKNOWN:0001",
  "gene": "UniProtKB:Q6ZN04",
  "gene_name": "RNA-binding protein MEX3B"
}